{
  "term_id": "UNKNOWN:0001",
  "gene_symbol": "SDK1",
  "gene_name": "Protein sidekick-1",
  "term_label": "Unknown molecular function",
  "gene": "UniProtKB:Q7Z5N4"
}